{
  "term_label": "proline dehydrogenase activity",
  "gene_name": "Proline dehydrogenase 1, mitochondrial",
  "gene_symbol": "PRODH",
  "gene": "UniProtKB:O43272",
  "term_id": "GO:0004657"
}